{
  "gene_name": "Probable ribonuclease ZC3H12B",
  "term_id": "GO:0004521",
  "gene_symbol": "ZC3H12B",
  "gene": "UniProtKB:Q5HYM0",
  "term_label": "RNA endonuclease activity"
}